{
  "term_id": "GO:0003980",
  "term_label": "UDP-glucose:glycoprotein glucosyltransferase activity",
  "gene_symbol": "UGGT2",
  "gene_name": "UDP-glucose:glycoprotein glucosyltransferase 2",
  "gene": "UniProtKB:Q9NYU1"
}